{
  "gene_name": "Plexin domain-containing protein 2",
  "term_id": "UNKNOWN:0003",
  "gene": "UniProtKB:Q6UX71",
  "term_label": "Unknown cellular component",
  "gene_symbol": "PLXDC2"
}